{
  "term_id": "UNKNOWN:0003",
  "gene_name": "Transmembrane protein 59-like",
  "gene_symbol": "TMEM59L",
  "gene": "UniProtKB:Q9UK28",
  "term_label": "Unknown cellular component"
}